detection of cytokinin stimulus [GO:0009722] (biological process) Relationships: is a type of detection of hormone stimulus [GO:0009720]; is a type of response to cytokinin [GO:0009735] Definition: The series of events in which a cytokinin stimulus is received by a cell and converted into a molecular signal. Sources: GOC:sm Also known as: perception of cytokinin stimulus